G protein-coupled purinergic nucleotide receptor activity [GO:0045028] (molecular function) References: PMID:9755289 Sources: GOC:mah Definition: Combining with a purine nucleotide and transmitting the signal across the membrane by activating an associated G-protein; promotes the exchange of GDP for GTP on the alpha subunit of a heterotrimeric G-protein complex. Also known as: G protein coupled purinergic nucleotide receptor activity, G-protein coupled purinergic nucleotide receptor activity, purinergic nucleotide receptor activity, G protein coupled, purinergic nucleotide receptor activity, G-protein coupled, P2Y, P2Y receptor Relationships: is a type of purinergic nucleotide receptor activity [GO:0001614]; is a type of GO:0004930; is part of GO:0035589 Subtypes: G protein-coupled ADP receptor activity [GO:0001621], cAMP receptor activity [GO:0001646], G protein-coupled ATP receptor activity [GO:0045031]